{
  "gene_symbol": "OR51I2",
  "term_label": "olfactory receptor activity",
  "gene_name": "Olfactory receptor 51I2",
  "gene": "UniProtKB:Q9H344",
  "term_id": "GO:0004984"
}